{
  "gene_name": "Serine protease hepsin",
  "gene": "UniProtKB:P05981",
  "gene_symbol": "HPN",
  "term_id": "GO:0005886",
  "term_label": "plasma membrane"
}